{
  "gene": "UniProtKB:Q9NYA1",
  "gene_name": "Sphingosine kinase 1",
  "gene_symbol": "SPHK1",
  "term_label": "cytoplasm",
  "term_id": "GO:0005737"
}